sorocarp development [GO:0030587] (biological process) Also known as: fruiting body development, fruiting body formation, sorocarp biosynthesis, sorocarp formation Definition: The process whose specific outcome is the progression of the sorocarp over time, from its formation to the mature structure. The process begins with the aggregation of individual cells and ends with the mature sorocarp. The sorocarp is a structure containing a spore-bearing sorus that sits on top of a stalk. An example of this process is found in Dictyostelium discoideum. Relationships: is a type of socially cooperative development [GO:0099120] Subtypes: chimeric sorocarp development [GO:0099134] Regulation: regulated by regulation of sorocarp development [GO:0031156] References: PMID:4332228 Sources: GOC:mah, GOC:mtg_sensu, ISBN:0521583640